{
  "gene_symbol": "LHFPL4",
  "gene_name": "LHFPL tetraspan subfamily member 4 protein",
  "term_id": "GO:0050811",
  "term_label": "GABA receptor binding",
  "gene": "UniProtKB:Q7Z7J7"
}